{
  "term_label": "cytoplasm",
  "gene": "UniProtKB:Q8WUJ0",
  "gene_name": "Serine_threonine_tyrosine-interacting protein",
  "term_id": "GO:0005737",
  "gene_symbol": "STYX"
}